{
  "term_id": "GO:0071203",
  "gene_name": "WAS_WASL-interacting protein family member 3",
  "gene_symbol": "WIPF3",
  "term_label": "WASH complex",
  "gene": "UniProtKB:A6NGB9"
}